{
  "term_label": "cytidine deaminase activity",
  "gene_symbol": "APOBEC3H",
  "gene": "UniProtKB:Q6NTF7",
  "term_id": "GO:0004126",
  "gene_name": "DNA dC-dU-editing enzyme APOBEC-3H"
}